{
  "gene_name": "Protein Largen",
  "gene_symbol": "PRR16",
  "gene": "UniProtKB:Q569H4",
  "term_label": "positive regulation of cell size",
  "term_id": "GO:0045793"
}